co-transcriptional gene silencing by RNA interference machinery [GO:0033562] (biological process) Definition: A process in which the RNAi machinery mediates the degradation of nascent transcripts in association with chromatin. Relationships: is a type of regulatory ncRNA-mediated gene silencing [GO:0031047] Also known as: RNAi-mediated CTGS, co-transcriptional gene silencing by small RNA, small RNA-mediated cotranscriptional gene silencing, cotranscriptional gene silencing by RNA interference machinery, cotranscriptional gene silencing by small RNA References: PMID:17512405, PMID:21151114, PMID:22431512 Sources: GOC:mah, GOC:vw